mannan binding [GO:2001065] (molecular function) Also known as: mannoglycan binding Definition: Binding to mannan. Relationships: is a type of GO:0030247 Sources: GOC:mengo_curators